{
  "gene_symbol": "ZNF449",
  "gene": "UniProtKB:Q6P9G9",
  "gene_name": "Zinc finger protein 449",
  "term_id": "GO:0000981",
  "term_label": "DNA-binding transcription factor activity, RNA polymerase II-specific"
}